{
  "gene_name": "Golgin subfamily A member 8T",
  "term_id": "GO:0000137",
  "gene": "UniProtKB:H3BQL2",
  "gene_symbol": "GOLGA8T",
  "term_label": "Golgi cis cisterna"
}